{
  "gene_symbol": "ZW10",
  "gene": "UniProtKB:O43264",
  "gene_name": "Centromere_kinetochore protein zw10 homolog",
  "term_label": "mitotic spindle assembly checkpoint signaling",
  "term_id": "GO:0007094"
}